{
  "gene_symbol": "REEP2",
  "term_label": "endoplasmic reticulum tubular network",
  "gene_name": "Receptor expression-enhancing protein 2",
  "term_id": "GO:0071782",
  "gene": "UniProtKB:Q9BRK0"
}